5-oxo-6E,8Z,11Z,14Z-icosatetraenoic acid binding [GO:0050646] (molecular function) Relationships: is a type of long-chain fatty acid binding [GO:0036041]; is a type of icosanoid binding [GO:0050542] Definition: Binding to 5-oxo-6E,8Z,11Z,14Z-icosatetraenoic acid, a straight-chain fatty acid with twenty carbon atoms and four double bonds. Sources: GOC:ai Also known as: 5-oxo-6E,8Z,11Z,14Z-eicosatetraenoic acid binding